ATPase-coupled monocarboxylic acid transmembrane transporter activity [GO:0033285] (MF) Sources: GOC:mlg Also known as: ATP-dependent monocarboxylic acid transmembrane transporter activity, monocarboxylic acid-transporting ATPase activity Definition: Enables the transfer of a solute or solutes from one side of a membrane to the other according to the reaction: ATP + H2O + monocarboxylic acid(out/in) = ADP + phosphate + monocarboxylic acid(in/out). Relationships: is a type of GO:0008028; is a type of GO:0033284 Subtypes: GO:0015432, ATPase-coupled ectoine transmembrane transporter activity [GO:0033286], ATPase-coupled hydroxyectoine transmembrane transporter activity [GO:0033288]